negative regulation of interleukin-6-mediated signaling pathway [GO:0070104] (biological process) Definition: Any process that decreases the rate, frequency or extent of an interleukin-6-mediated signaling pathway. Sources: GOC:BHF, GOC:mah Also known as: negative regulation of IL-6-mediated signaling pathway, negative regulation of interleukin-6-mediated signalling pathway Relationships: is a type of negative regulation of cytokine-mediated signaling pathway [GO:0001960]; is a type of regulation of interleukin-6-mediated signaling pathway [GO:0070103]; negatively regulates interleukin-6-mediated signaling pathway [GO:0070102]